alkanesulfonate transmembrane transport [GO:0042918] (biological process) References: PMID:31802112 Subtypes: taurine transmembrane transport [GO:0015734] Relationships: is a type of GO:0015711; is a type of organic acid transport [GO:0015849]; is a type of transmembrane transport [GO:0055085]; is a type of sulfur compound transport [GO:0072348] Definition: The directed movement of an alkanesulfonate into, out of or within a cell, or between cells, by means of some agent such as a transporter or pore. Alkanesulfonates are organic esters or salts of sulfonic acid containing an aliphatic hydrocarbon radical. Also known as: alkanesulfonate transport, alkanesulphonate transport